positive regulation of myeloid progenitor cell differentiation [GO:1905455] (biological process) References: PMID:27010503 Sources: GOC:TermGenie, GO_REF:0000058 Definition: Any process that activates or increases the frequency, rate or extent of myeloid progenitor cell differentiation. Relationships: is a type of GO:1901534; is a type of regulation of myeloid progenitor cell differentiation [GO:1905453]; positively regulates myeloid progenitor cell differentiation [GO:0002318] Also known as: up regulation of myeloid progenitor cell differentiation, up-regulation of myeloid progenitor cell differentiation, upregulation of myeloid progenitor cell differentiation, activation of myeloid progenitor cell differentiation